{
  "gene": "UniProtKB:O95868",
  "term_label": "acetylcholine receptor signaling pathway",
  "gene_name": "Lymphocyte antigen 6 complex locus protein G6d",
  "gene_symbol": "LY6G6D",
  "term_id": "GO:0095500"
}